negative regulation of estrogen secretion [GO:2000862] (biological process) Also known as: negative regulation of oestrogen secretion Relationships: is a type of GO:2000832; is_a regulation of estrogen secretion [GO:2000861]; negatively regulates estrogen secretion [GO:0035937] Sources: GOC:sl Definition: Any process that stops, prevents or reduces the frequency, rate or extent of estrogen secretion.